{
  "term_label": "regulation of transcription by RNA polymerase II",
  "term_id": "GO:0006357",
  "gene": "UniProtKB:Q70SY1",
  "gene_name": "Cyclic AMP-responsive element-binding protein 3-like protein 2",
  "gene_symbol": "CREB3L2"
}